{
  "term_label": "Unknown molecular function",
  "gene_symbol": "ODAD1",
  "term_id": "UNKNOWN:0001",
  "gene_name": "Outer dynein arm-docking complex subunit 1",
  "gene": "UniProtKB:Q96M63"
}